response to chlorate [GO:0010157] (biological process) Sources: GOC:sm Subtypes: GO:0071246 Relationships: is a type of response to oxygen-containing compound [GO:1901700] Definition: Any process that results in a change in state or activity of a cell or an organism (in terms of movement, secretion, enzyme production, gene expression, etc.) as a result of a chlorate stimulus.